{
  "term_label": "microtubule cytoskeleton",
  "gene_symbol": "TEKT2",
  "term_id": "GO:0015630",
  "gene_name": "Tektin-2",
  "gene": "UniProtKB:Q9UIF3"
}